{
  "term_label": "regulation of DNA repair",
  "gene_symbol": "RADX",
  "term_id": "GO:0006282",
  "gene": "UniProtKB:Q6NSI4",
  "gene_name": "RPA-related protein RADX"
}